{
  "term_id": "GO:0005178",
  "gene_name": "CCN family member 2",
  "gene": "UniProtKB:P29279",
  "term_label": "integrin binding",
  "gene_symbol": "CCN2"
}